dendritic spine neck [GO:0044326] (CC) Relationships: is a type of GO:0110165; is part of dendritic spine [GO:0043197] Sources: GOC:nln Also known as: neck, spine neck, pedicle Definition: Part of the dendritic spine that connects the dendritic shaft to the head of the dendritic spine.